{
  "gene_symbol": "XPC",
  "gene_name": "DNA repair protein complementing XP-C cells",
  "term_label": "cytoplasm",
  "term_id": "GO:0005737",
  "gene": "UniProtKB:Q01831"
}